negative regulation of sorocarp spore cell differentiation [GO:1901262] (biological process) Sources: GOC:TermGenie, GOC:rjd Definition: Any process that stops, prevents or reduces the frequency, rate or extent of sorocarp spore cell differentiation. Also known as: down regulation of sorocarp spore cell differentiation, down-regulation of sorocarp spore cell differentiation, downregulation of sorocarp spore cell differentiation, inhibition of sorocarp spore cell differentiation Relationships: is a type of GO:0045596; is a type of regulation of sorocarp spore cell differentiation [GO:1901261]; negatively regulates sorocarp spore cell differentiation [GO:0044671]